transcription preinitiation complex [GO:0097550] (cellular component) Relationships: is_a protein-DNA complex [GO:0032993] Definition: A protein-DNA complex composed of proteins binding promoter DNA to form the transcriptional preinitiation complex (PIC), the formation of which is a prerequisite for transcription. References: PMID:22751016 Sources: GOC:di Also known as: DNA-templated transcriptional preinitiation complex, transcriptional pre-initiation complex, transcriptional preinitiation complex, PIC, preinitiation complex